prostate gland development [GO:0030850] (biological process) Relationships: is a type of GO:0048608; is a type of gland development [GO:0048732]; is part of urogenital system development [GO:0001655] References: PMID:11839751 Definition: The process whose specific outcome is the progression of the prostate gland over time, from its formation to the mature structure. The prostate gland is a partly muscular, partly glandular body that is situated near the base of the mammalian male urethra and secretes an alkaline viscid fluid which is a major constituent of the ejaculatory fluid. Also known as: prostate development